{
  "gene_symbol": "PPIH",
  "gene_name": "Peptidyl-prolyl cis-trans isomerase H",
  "gene": "UniProtKB:O43447",
  "term_id": "GO:0003755",
  "term_label": "peptidyl-prolyl cis-trans isomerase activity"
}